glutathione-regulated potassium exporter activity [GO:0015503] (molecular function) Definition: Enables the transfer of a solute or solutes from one side of a membrane to the other according to the reaction: K+(in) + H+(out) = K+(out) + H+(in), where glutathione maintains the closed state. Relationships: is a type of GO:0022821 References: PMID:11053405 Sources: TC:2.A.37.1.1, TC:2.A.37.1.2